{
  "gene_name": "Claudin-20",
  "gene_symbol": "CLDN20",
  "term_id": "UNKNOWN:0002",
  "term_label": "Unknown biological process",
  "gene": "UniProtKB:P56880"
}